{
  "gene_name": "PRKC apoptosis WT1 regulator protein",
  "gene_symbol": "PAWR",
  "gene": "UniProtKB:Q96IZ0",
  "term_id": "UNKNOWN:0001",
  "term_label": "Unknown molecular function"
}